{
  "gene_name": "Arf-GAP with GTPase, ANK repeat and PH domain-containing protein 2",
  "term_id": "GO:0005634",
  "gene_symbol": "AGAP2",
  "term_label": "nucleus",
  "gene": "UniProtKB:Q99490"
}